membranous septum morphogenesis [GO:0003149] (biological process) Definition: The process in which the membranous septum is generated and organized. The membranous septum is the upper part of ventricular septum. Sources: GOC:mtg_heart Relationships: is a type of GO:0009653; is part of ventricular septum morphogenesis [GO:0060412]